{
  "gene_name": "Cryptochrome-2",
  "gene": "UniProtKB:Q49AN0",
  "term_id": "GO:0005634",
  "term_label": "nucleus",
  "gene_symbol": "CRY2"
}